{
  "gene_symbol": "EPYC",
  "gene_name": "Epiphycan",
  "gene": "UniProtKB:Q99645",
  "term_label": "bone development",
  "term_id": "GO:0060348"
}